anthranilate-CoA ligase activity [GO:0018860] (molecular function) Also known as: anthranilate--CoA ligase activity, 2-aminobenzoate coenzyme A ligase activity, 2-aminobenzoate-CoA ligase activity, 2-aminobenzoate-coenzyme A ligase activity, anthranilate:CoA ligase (AMP-forming), anthraniloyl coenzyme A synthetase activity Relationships: is_a CoA-ligase activity [GO:0016405]; is a type of GO:0016878 Definition: Catalysis of the reaction: ATP + anthranilate + CoA = AMP + diphosphate + anthranilyl-CoA. Sources: EC:6.2.1.32